regulation of serotonin uptake [GO:0051611] (biological process) Definition: Any process that modulates the frequency, rate or extent of the directed movement of the monoamine neurotransmitter serotonin into a cell. Relationships: is a type of regulation of neurotransmitter uptake [GO:0051580]; regulates serotonin uptake [GO:0051610] Also known as: regulation of 5-HT uptake, regulation of 5-hydroxytryptamine uptake, regulation of 5HT uptake, regulation of serotonin import Sources: GOC:ai Subtypes: GO:0051612, positive regulation of serotonin uptake [GO:0051613]